{
  "gene_symbol": "CCDC152",
  "gene_name": "Coiled-coil domain-containing protein 152",
  "gene": "UniProtKB:Q4G0S7",
  "term_id": "UNKNOWN:0001",
  "term_label": "Unknown molecular function"
}